{
  "gene_symbol": "RNF113A",
  "term_id": "GO:0000398",
  "gene_name": "E3 ubiquitin-protein ligase RNF113A",
  "gene": "UniProtKB:O15541",
  "term_label": "mRNA splicing, via spliceosome"
}